{
  "term_label": "Unknown cellular component",
  "gene": "UniProtKB:Q70EK9",
  "term_id": "UNKNOWN:0003",
  "gene_name": "Ubiquitin carboxyl-terminal hydrolase 51",
  "gene_symbol": "USP51"
}